CENP-A containing nucleosome [GO:0043505] (cellular component) Also known as: CENP-S-T-W-X, CNP-T-W-S-X complex, CenH3 containing nucleosome, centromere specific nucleosome, centromere-specific nucleosome, centromeric nucleosome References: PMID:15175412, PMID:16183641 Sources: GOC:go_curators Relationships: is_a nucleosome [GO:0000786]; is part of GO:0061638 Definition: A form of nucleosome located only at the centromere, in which the histone H3 is replaced by the variant form CENP-A (sometimes known as CenH3).